regulation of signaling [GO:0023051] (biological process) Sources: GOC:mtg_signal Relationships: is a type of regulation of biological process [GO:0050789]; regulates signaling [GO:0023052] Also known as: regulation of signaling process, regulation of signalling process Definition: Any process that modulates the frequency, rate or extent of a signaling process. Subtypes: GO:0001919, GO:0009966, GO:0023056, negative regulation of signaling [GO:0023057], GO:0046883, GO:0061356, regulation of c-di-GMP signaling [GO:0061940], GO:0099177, regulation of synaptic signaling by nitric oxide [GO:0150045], regulation of trichome patterning [GO:1900032], GO:2001284